{
  "gene": "UniProtKB:Q8WXB1",
  "gene_symbol": "METTL21A",
  "term_id": "GO:0016279",
  "gene_name": "Protein N-lysine methyltransferase METTL21A",
  "term_label": "protein-lysine N-methyltransferase activity"
}